hydrogen peroxide catabolic process [GO:0042744] (BP) Sources: GOC:jl Relationships: is a type of GO:0009056; is a type of GO:0042743 Also known as: H2O2 catabolic process, hydrogen peroxide breakdown, hydrogen peroxide catabolism, hydrogen peroxide degradation, H2O2 scavenging, detoxification of H2O2, detoxification of hydrogen peroxide, hydrogen peroxide removal, hydrogen peroxide scavenging Regulation: positively regulated by positive regulation of hydrogen peroxide catabolic process [GO:1903285]; RO_0002211 by regulation of hydrogen peroxide catabolic process [GO:2000295]; negatively regulated by GO:2000296 Definition: The chemical reactions and pathways resulting in the breakdown of hydrogen peroxide (H2O2). Subtypes: ascorbate glutathione cycle [GO:0033355]